tetrapyrrole catabolic process [GO:0033015] (biological process) Subtypes: GO:0006787, cobalamin catabolic process [GO:0042366], GO:0046141 Sources: GOC:mah Relationships: is a type of GO:0009056; is a type of tetrapyrrole metabolic process [GO:0033013] Regulation: regulated by regulation of tetrapyrrole catabolic process [GO:1901404]; RO_0002212 by negative regulation of tetrapyrrole catabolic process [GO:1901405]; positively regulated by positive regulation of tetrapyrrole catabolic process [GO:1901406] Definition: The chemical reactions and pathways leading to the breakdown of tetrapyrroles, natural pigments containing four pyrrole rings joined by one-carbon units linking position 2 of one pyrrole ring to position 5 of the next. Also known as: tetrapyrrole breakdown, tetrapyrrole catabolism, tetrapyrrole degradation